{
  "gene": "UniProtKB:Q9Y4Z2",
  "term_label": "axon development",
  "gene_name": "Neurogenin-3",
  "gene_symbol": "NEUROG3",
  "term_id": "GO:0061564"
}